{
  "gene_name": "Homeobox protein Hox-A2",
  "gene": "UniProtKB:O43364",
  "term_label": "nucleus",
  "gene_symbol": "HOXA2",
  "term_id": "GO:0005634"
}